{
  "gene_symbol": "CALML6",
  "term_label": "cytoplasm",
  "gene_name": "Calmodulin-like protein 6",
  "term_id": "GO:0005737",
  "gene": "UniProtKB:Q8TD86"
}